neurohypophysis development [GO:0021985] (BP) Also known as: neurophysis development, posterior pituitary development, posterior pituitary gland development Relationships: is a type of GO:0048732; is part of GO:0021983 Definition: The progression of the neurohypophysis over time from its initial formation until its mature state. The neurohypophysis is the part of the pituitary gland that secretes hormones involved in blood pressure regulation. Sources: GOC:cls, GOC:dgh, GOC:dph, GOC:jid, GO_REF:0000021